{
  "term_id": "GO:0012505",
  "gene_symbol": "STX4",
  "gene": "UniProtKB:Q12846",
  "term_label": "endomembrane system",
  "gene_name": "Syntaxin-4"
}